microtubule-dependent intracellular transport of viral material towards nucleus [GO:0075521] (biological process) Sources: UniProtKB-KW:KW-1177, VZ:983 Definition: The directed movement of a virus, or part of a virus, towards the host cell nucleus using host microtubules. Also known as: microtubule-dependent intracellular transport of viral material to nucleus Relationships: is a type of GO:0075519; is_a transport of viral material towards nucleus [GO:0075606]